{
  "gene_symbol": "UGT2A3",
  "term_id": "UNKNOWN:0003",
  "gene_name": "UDP-glucuronosyltransferase 2A3",
  "term_label": "Unknown cellular component",
  "gene": "UniProtKB:Q6UWM9"
}